{
  "term_label": "nucleus",
  "gene": "UniProtKB:Q9NVV9",
  "term_id": "GO:0005634",
  "gene_symbol": "THAP1",
  "gene_name": "THAP domain-containing protein 1"
}